{
  "gene": "UniProtKB:O15467",
  "term_id": "GO:0008009",
  "gene_name": "C-C motif chemokine 16",
  "gene_symbol": "CCL16",
  "term_label": "chemokine activity"
}